{
  "term_id": "UNKNOWN:0001",
  "gene_name": "Interferon-inducible GTPase 5",
  "term_label": "Unknown molecular function",
  "gene_symbol": "IRGC",
  "gene": "UniProtKB:Q6NXR0"
}